prolactin secreting cell differentiation [GO:0060127] (biological process) Sources: GOC:dph Relationships: is a type of cell differentiation [GO:0030154]; is part of adenohypophysis development [GO:0021984] Definition: The process in which a relatively unspecialized cell acquires specialized structural and/or functional features of a prolactin secreting cell. A prolactin secreting cell is an acidophilic cell of the anterior pituitary that produces prolactin. Also known as: epsilon-acidophil differentiation, lactotrope differentiation, lactotroph differentiation, lactotropic cell differentiation, mammotrope differentiation, mammotroph differentiation, mammotrophic cell differentiation, mammotropic cell differentiation